tellurite transmembrane transporter activity [GO:0015654] (molecular function) Definition: Enables the transfer of tellurite from one side of a membrane to the other. Tellurite is a salt of tellurous acid or an oxide of tellurium which occurs sparingly in tufts of white or yellowish crystals. Relationships: is a type of GO:0022857 Also known as: tellurite uptake transmembrane transporter activity, tellurite-resistance uptake permease activity, tellurite-resistance uptake transmembrane transporter activity Sources: GOC:ai